{
  "term_id": "GO:0098793",
  "term_label": "presynapse",
  "gene": "UniProtKB:Q99962",
  "gene_symbol": "SH3GL2",
  "gene_name": "Endophilin-A1"
}